{
  "gene": "UniProtKB:Q05066",
  "term_id": "GO:0030154",
  "gene_name": "Sex-determining region Y protein",
  "term_label": "cell differentiation",
  "gene_symbol": "SRY"
}